{
  "term_label": "collagen fibril organization",
  "gene": "UniProtKB:P02461",
  "gene_name": "Collagen alpha-1(III) chain",
  "term_id": "GO:0030199",
  "gene_symbol": "COL3A1"
}